lariciresinol reductase activity [GO:0010284] (molecular function) Definition: Catalysis of the reaction: lariciresinol + NADPH + H+ = secoisolariciresinol + NADP+. References: PMID:10066819, PMID:7592828 Relationships: is a type of GO:0120546